{
  "gene_name": "Kelch-like protein 40",
  "gene_symbol": "KLHL40",
  "gene": "UniProtKB:Q2TBA0",
  "term_id": "GO:0032435",
  "term_label": "negative regulation of proteasomal ubiquitin-dependent protein catabolic process"
}